{
  "gene": "UniProtKB:Q9NQ90",
  "gene_symbol": "ANO2",
  "term_id": "GO:0005886",
  "term_label": "plasma membrane",
  "gene_name": "Anoctamin-2"
}